glycyrrhizinate beta-glucuronidase activity [GO:0047967] (molecular function) Also known as: glycyrrhizinate b-glucuronidase activity, glycyrrhizin beta-hydrolase activity, glycyrrhizin hydrolase activity, glycyrrhizinate glucuronosylhydrolase activity, glycyrrhizinic acid hydrolase activity Definition: Catalysis of the reaction: glycyrrhizate + H2O = 2-(beta-D-glucuronosyl)-D-glucuronate + glycyrrhetinate. Sources: EC:3.2.1.128, RHEA:17369 Relationships: is a type of GO:0046574